response to TNF agonist [GO:0061481] (biological process) Definition: Any process that results in a change in state or activity of a cell or an organism (in terms of movement, secretion, enzyme production, gene expression, etc.) as a result of a TNF agonist stimulus. Relationships: is a type of GO:0042221 Sources: GOC:dph